brefeldin A esterase activity [GO:0052772] (molecular function) Definition: Catalysis of the hydrolysis of brefeldin A to produce brefeldin A acid. Brefeldin A is also known as gamma,4-dihydroxy-2-(6-hydroxy-1-heptenyl)-4-cyclopentanecrotonic acid lambda-lactone. References: PMID:10201402, PMID:8106385 Sources: GOC:mengo_curators Also known as: BFA esterase activity, brefeldin A hydrolase activity Relationships: is a type of carboxylic ester hydrolase activity [GO:0052689]